{
  "term_label": "Fc-epsilon receptor I complex",
  "term_id": "GO:0032998",
  "gene_symbol": "MS4A2",
  "gene_name": "High affinity immunoglobulin epsilon receptor subunit beta",
  "gene": "UniProtKB:Q01362"
}